{
  "term_label": "endopeptidase activity",
  "gene": "UniProtKB:Q96LU5",
  "term_id": "GO:0004175",
  "gene_symbol": "IMMP1L",
  "gene_name": "Mitochondrial inner membrane protease subunit 1"
}